{
  "gene_symbol": "ERVK-11",
  "gene": "UniProtKB:Q9UQG0",
  "gene_name": "Endogenous retrovirus group K member 11 Pol protein",
  "term_id": "UNKNOWN:0002",
  "term_label": "Unknown biological process"
}